phytyl-P kinase activity [GO:0102763] (molecular function) Definition: Catalysis of the reaction: a ribonucleoside 5'-triphosphate + phytyl phosphate = a ribonucleoside 5'-diphosphate + phytyl diphosphate. Relationships: is a type of phosphotransferase activity, phosphate group as acceptor [GO:0016776] Sources: RHEA:38099